{
  "gene": "UniProtKB:Q5VU65",
  "term_label": "Unknown biological process",
  "term_id": "UNKNOWN:0002",
  "gene_name": "Nuclear pore membrane glycoprotein 210-like",
  "gene_symbol": "NUP210L"
}